{
  "gene_name": "PALM2 and AKAP2 fusion",
  "gene_symbol": "PALM2AKAP2",
  "term_label": "Unknown biological process",
  "term_id": "UNKNOWN:0002",
  "gene": "UniProtKB:C9JA33"
}